compound eye cone cell fate determination [GO:0042680] (biological process) Sources: GOC:mtg_sensu Definition: The process in which a cell becomes capable of differentiating autonomously into a compound eye cone cell regardless of its environment; upon determination, the cell fate cannot be reversed. Relationships: is a type of cell fate determination [GO:0001709]; BFO_0000050 GO:0042676